embryonic limb morphogenesis [GO:0030326] (biological process) Sources: GOC:bf, GOC:jl, ISBN:0395825172 Subtypes: embryonic forelimb morphogenesis [GO:0035115], GO:0035116 Definition: The process, occurring in the embryo, by which the anatomical structures of the limb are generated and organized. A limb is an appendage of an animal used for locomotion or grasping. Relationships: is a type of limb morphogenesis [GO:0035108]; is a type of GO:0035113